positive regulation of mineralocorticoid secretion [GO:2000857] (biological process) Relationships: is a type of positive regulation of corticosteroid hormone secretion [GO:2000848]; is_a regulation of mineralocorticoid secretion [GO:2000855]; positively regulates mineralocorticoid secretion [GO:0035931] Subtypes: positive regulation of aldosterone secretion [GO:2000860] Definition: Any process that activates or increases the frequency, rate or extent of mineralocorticoid secretion. Sources: GOC:sl